respiratory gaseous exchange by respiratory system [GO:0007585] (biological process) Also known as: breathing, respiration Regulation: regulated by regulation of respiratory gaseous exchange [GO:0043576]; negatively regulated by GO:1903941; positively regulated by positive regulation of respiratory gaseous exchange [GO:1903942] Definition: The process of gaseous exchange between an organism and its environment. In plants, microorganisms, and many small animals, air or water makes direct contact with the organism's cells or tissue fluids, and the processes of diffusion supply the organism with dioxygen (O2) and remove carbon dioxide (CO2). In larger animals the efficiency of gaseous exchange is improved by specialized respiratory organs, such as lungs and gills, which are ventilated by breathing mechanisms. Sources: ISBN:0198506732 Relationships: is a type of multicellular organismal process [GO:0032501]